sucrose mediated signaling [GO:0009745] (BP) Also known as: sucrose mediated signalling Definition: The series of molecular signals mediated by the detection of sucrose. Relationships: is a type of sugar mediated signaling pathway [GO:0010182]; is part of cellular response to sucrose stimulus [GO:0071329] Sources: GOC:sm